{
  "gene_name": "Hemoglobin subunit mu",
  "term_label": "erythrocyte development",
  "gene_symbol": "HBM",
  "term_id": "GO:0048821",
  "gene": "UniProtKB:Q6B0K9"
}